{
  "term_label": "Unknown cellular component",
  "gene": "UniProtKB:Q9P281",
  "gene_name": "BAH and coiled-coil domain-containing protein 1",
  "gene_symbol": "BAHCC1",
  "term_id": "UNKNOWN:0003"
}